{
  "term_id": "GO:0002860",
  "gene": "UniProtKB:O95727",
  "gene_name": "Cytotoxic and regulatory T-cell molecule",
  "gene_symbol": "CRTAM",
  "term_label": "positive regulation of natural killer cell mediated cytotoxicity directed against tumor cell target"
}